{
  "term_id": "GO:0005737",
  "gene_name": "Myotubularin-related protein 4",
  "term_label": "cytoplasm",
  "gene": "UniProtKB:Q9NYA4",
  "gene_symbol": "MTMR4"
}